{
  "term_id": "GO:0001819",
  "gene_symbol": "IL21",
  "term_label": "positive regulation of cytokine production",
  "gene_name": "Interleukin-21",
  "gene": "UniProtKB:Q9HBE4"
}